{
  "gene": "UniProtKB:O15169",
  "gene_name": "Axin-1",
  "term_label": "ubiquitin protein ligase binding",
  "gene_symbol": "AXIN1",
  "term_id": "GO:0031625"
}